reelin complex [GO:0110157] (CC) Definition: An extracellular complex that binds lipoprotein receptors VLDLR and APOER2, cadherin-related neuronal receptors (CNRs) or alpha3beta1 integrin and induces various downstream, reelin-dependent, phosphorylation cascades. It ultimately affects polarization, differentiation, neuronal migration and layer formation in the embryonic brain and neuron growth, maturation, and synaptic activity in the postnatal and adult brain. References: PMID:21844191, PMID:28887403 Sources: GOC:bhm Relationships: is a type of GO:0032991; is part of GO:0005615